extrinsic component of organelle membrane [GO:0031312] (cellular component) Subtypes: extrinsic component of intraperoxisomal membrane [GO:0005780], GO:0031313, GO:0031314, extrinsic component of mitochondrial outer membrane [GO:0031315], GO:0031316, extrinsic component of plastid membrane [GO:0035452], GO:0042406, extrinsic component of Golgi membrane [GO:0090498], GO:0097629, GO:0097632, GO:0098850, GO:0098922 Also known as: extrinsic to organelle membrane Relationships: is a type of GO:0019898; is part of organelle membrane [GO:0031090]; BFO_0000050 GO:0043229 Definition: The component of an organelle membrane consisting of gene products and protein complexes that are loosely bound to one of its surfaces, but not integrated into the hydrophobic region. Sources: GOC:dos, GOC:mah